{
  "gene": "UniProtKB:A0A1B0GVY4",
  "gene_symbol": "SMIM31",
  "term_id": "UNKNOWN:0002",
  "term_label": "Unknown biological process",
  "gene_name": "Small integral membrane protein 31"
}